{
  "gene": "UniProtKB:P07333",
  "gene_name": "Macrophage colony-stimulating factor 1 receptor",
  "term_id": "GO:0005886",
  "term_label": "plasma membrane",
  "gene_symbol": "CSF1R"
}